{
  "gene_name": "Olfactory receptor 1L1",
  "gene_symbol": "OR1L1",
  "gene": "UniProtKB:Q8NH94",
  "term_id": "GO:0007165",
  "term_label": "signal transduction"
}